{
  "term_label": "neuron differentiation",
  "gene_symbol": "VXN",
  "term_id": "GO:0030182",
  "gene": "UniProtKB:Q8TAG6",
  "gene_name": "Vexin"
}